{
  "gene": "UniProtKB:Q9NUS5",
  "gene_name": "AP-5 complex subunit sigma-1",
  "term_label": "AP-type membrane coat adaptor complex",
  "gene_symbol": "AP5S1",
  "term_id": "GO:0030119"
}